{
  "gene_symbol": "USP26",
  "gene": "UniProtKB:Q9BXU7",
  "term_label": "nucleus",
  "term_id": "GO:0005634",
  "gene_name": "Ubiquitin carboxyl-terminal hydrolase 26"
}